{
  "gene": "UniProtKB:Q9Y2C9",
  "gene_symbol": "TLR6",
  "gene_name": "Toll-like receptor 6",
  "term_id": "GO:0071723",
  "term_label": "lipopeptide binding"
}